{
  "gene_name": "Zinc finger and BTB domain-containing protein 20",
  "term_label": "RNA polymerase II cis-regulatory region sequence-specific DNA binding",
  "gene": "UniProtKB:Q9HC78",
  "term_id": "GO:0000978",
  "gene_symbol": "ZBTB20"
}